thyroid hormone catabolic process [GO:0042404] (biological process) Definition: The chemical reactions and pathways resulting in the breakdown of any of the compounds secreted by the thyroid gland, largely thyroxine and triiodothyronine. Also known as: thyroid hormone breakdown, thyroid hormone catabolism, thyroid hormone degradation Sources: GOC:jl, ISBN:0198506732 Relationships: is a type of phenol-containing compound catabolic process [GO:0019336]; is a type of GO:0042219; is a type of GO:0042403; is_a GO:0042447